{
  "term_id": "GO:0009653",
  "gene_symbol": "FOXQ1",
  "term_label": "anatomical structure morphogenesis",
  "gene": "UniProtKB:Q9C009",
  "gene_name": "Forkhead box protein Q1"
}